{
  "term_label": "nucleus",
  "gene": "UniProtKB:Q9Y615",
  "gene_name": "Actin-like protein 7A",
  "term_id": "GO:0005634",
  "gene_symbol": "ACTL7A"
}